{
  "gene_name": "Ephrin-B3",
  "gene_symbol": "EFNB3",
  "term_label": "ephrin receptor binding",
  "gene": "UniProtKB:Q15768",
  "term_id": "GO:0046875"
}